{
  "gene_name": "Kinesin-like protein KIF13B",
  "term_label": "microtubule-based movement",
  "gene": "UniProtKB:Q9NQT8",
  "gene_symbol": "KIF13B",
  "term_id": "GO:0007018"
}